lactosylceramide alpha-2,3-sialyltransferase activity [GO:0047291] (molecular function) Also known as: CMP-acetylneuraminate-lactosylceramide-sialyltransferase, cytidine monophosphoacetylneuraminate-lactosylceramide sialyltransferase, GM3 synthase activity, cytidine monophosphoacetylneuraminate-lactosylceramide alpha2,3- sialyltransferase activity, ganglioside GM3 synthase activity Sources: EC:2.4.3.9, MetaCyc:2.4.99.9-RXN Definition: Catalysis of the reaction: cytolipin-H + CMP-N-acetylneuraminate = alpha-N-acetylneuraminyl-2,3-beta-D-galactosyl-1,4-beta-D-glucosylceramide + CMP. Alpha-N-acetylneuraminyl-2,3-beta-D-galactosyl-1,4-beta-D-glucosylceramide is also known as GM3. Relationships: is a type of sialyltransferase activity [GO:0008373]